{
  "gene_symbol": "NKX2-1",
  "gene": "UniProtKB:P43699",
  "gene_name": "Homeobox protein Nkx-2.1",
  "term_label": "cell differentiation",
  "term_id": "GO:0030154"
}